{
  "term_label": "Unknown cellular component",
  "gene_name": "FHF complex subunit HOOK-interacting protein 1A",
  "term_id": "UNKNOWN:0003",
  "gene": "UniProtKB:Q05DH4",
  "gene_symbol": "FHIP1A"
}